{
  "term_label": "Unknown cellular component",
  "term_id": "UNKNOWN:0003",
  "gene_name": "POU class 2 homeobox associating factor 3",
  "gene": "UniProtKB:A8K830",
  "gene_symbol": "POU2AF3"
}